{
  "gene": "UniProtKB:Q8N196",
  "gene_name": "Homeobox protein SIX5",
  "gene_symbol": "SIX5",
  "term_id": "GO:0005634",
  "term_label": "nucleus"
}